{
  "term_id": "GO:0042761",
  "gene_name": "Very-long-chain enoyl-CoA reductase",
  "gene_symbol": "TECR",
  "gene": "UniProtKB:Q9NZ01",
  "term_label": "very long-chain fatty acid biosynthetic process"
}